{
  "term_label": "protein folding chaperone",
  "gene_name": "PAT complex subunit Asterix",
  "gene_symbol": "WDR83OS",
  "gene": "UniProtKB:Q9Y284",
  "term_id": "GO:0044183"
}